{
  "gene_symbol": "PTGDS",
  "term_id": "UNKNOWN:0002",
  "gene_name": "Prostaglandin-H2 D-isomerase",
  "gene": "UniProtKB:P41222",
  "term_label": "Unknown biological process"
}